{
  "gene_name": "Microtubule organization protein AKNA",
  "gene_symbol": "AKNA",
  "term_id": "GO:0001837",
  "term_label": "epithelial to mesenchymal transition",
  "gene": "UniProtKB:Q7Z591"
}